{
  "term_id": "GO:0090263",
  "gene_symbol": "TNKS2",
  "gene": "UniProtKB:Q9H2K2",
  "term_label": "positive regulation of canonical Wnt signaling pathway",
  "gene_name": "Poly [ADP-ribose] polymerase tankyrase-2"
}